{
  "term_id": "GO:0007519",
  "gene_name": "Myosin regulatory light chain 11",
  "gene_symbol": "MYL11",
  "gene": "UniProtKB:Q96A32",
  "term_label": "skeletal muscle tissue development"
}